post-embryonic eye morphogenesis [GO:0048050] (biological process) Sources: GOC:jid, GOC:sensu Relationships: is a type of eye morphogenesis [GO:0048592] Subtypes: post-embryonic camera-type eye morphogenesis [GO:0048597] Definition: The process, occurring after embryonic development, by which the anatomical structures of the eye are generated and organized. The eye is the organ of sight.